{
  "term_label": "nucleus",
  "gene_name": "Homeobox and leucine zipper protein Homez",
  "term_id": "GO:0005634",
  "gene_symbol": "HOMEZ",
  "gene": "UniProtKB:Q8IX15"
}